thromboxane-A synthase activity [GO:0004796] (MF) Definition: Catalysis of the reaction: prostaglandin H(2) = thromboxane A(2). Sources: EC:5.3.99.5, RHEA:17137 Also known as: cytochrome P450 CYP5, (5Z,13E)-(15S)-9alpha,11alpha-epidioxy-15-hydroxyprosta-5,13-dienoate isomerase activity, (5Z,13E)-(15S)-9alpha,11alpha-epidioxy-15-hydroxyprosta-5,13-dienoate thromboxane-A2-isomerase activity, thromboxane synthase activity, thromboxane synthetase activity Relationships: is a type of GO:0016860